cell morphogenesis involved in Malpighian tubule morphogenesis [GO:0061336] (biological process) References: PMID:19783135 Sources: GOC:dph, GOC:mtg_kidney_jan10 Relationships: is a type of cell morphogenesis [GO:0000902]; BFO_0000050 Malpighian tubule morphogenesis [GO:0007443] Definition: The shape change of an epithelial cell from a columnar to squamous cell morphology that contributes to the shaping of the Malpighian tubule.